{
  "gene_symbol": "CPSF7",
  "gene": "UniProtKB:Q8N684",
  "term_label": "mRNA cleavage and polyadenylation specificity factor complex",
  "gene_name": "Cleavage and polyadenylation specificity factor subunit 7",
  "term_id": "GO:0005847"
}